L-gamma-glutamyl-L-propargylglycine hydroxylase activity [GO:0062148] (MF) Definition: Catalysis of the reaction: 2-oxoglutarate + L-gamma-glutamyl-L-propargylglycine + O2 = CO2 + L-gamma-glutamyl-(3R)-L-beta-ethynylserine + succinate. References: PMID:30867596 Sources: RHEA:59900 Relationships: is a type of GO:0016706